L-lysine efflux transmembrane transporter activity [GO:0015661] (molecular function) Sources: GOC:ai, GOC:mtg_transport, ISBN:0815340729 Definition: Enables the transfer of L-lysine from the inside of the cell to the outside of the cell across a membrane. Also known as: L-lysine exporter activity, L-lysine, 2,6-diaminohexanoic acid efflux transmembrane transporter activity Relationships: is a type of GO:0015189; is a type of L-amino acid efflux transmembrane transporter activity [GO:0034639]